{
  "gene": "UniProtKB:Q5R3I4",
  "gene_name": "Tetratricopeptide repeat protein 38",
  "gene_symbol": "TTC38",
  "term_label": "Unknown molecular function",
  "term_id": "UNKNOWN:0001"
}